{
  "term_id": "GO:0016192",
  "gene": "UniProtKB:Q96KC2",
  "gene_name": "ADP-ribosylation factor-like protein 5B",
  "term_label": "vesicle-mediated transport",
  "gene_symbol": "ARL5B"
}